{
  "gene": "UniProtKB:O60287",
  "term_id": "GO:0005730",
  "gene_name": "Nucleolar pre-ribosomal-associated protein 1",
  "term_label": "nucleolus",
  "gene_symbol": "URB1"
}